negative regulation of seed dormancy process [GO:1902039] (biological process) Also known as: down regulation of seed dormancy process, down-regulation of seed dormancy process, downregulation of seed dormancy process, inhibition of seed dormancy process, down regulation of seed dormancy, down-regulation of seed dormancy, downregulation of seed dormancy, inhibition of seed dormancy, negative regulation of seed dormancy Definition: Any process that stops, prevents or reduces the frequency, rate or extent of seed dormancy process. Relationships: is a type of negative regulation of developmental process [GO:0051093]; is a type of negative regulation of multicellular organismal process [GO:0051241]; is_a regulation of seed dormancy process [GO:2000033]; is_a negative regulation of reproductive process [GO:2000242]; negatively regulates seed dormancy process [GO:0010162] References: PMID:23378449 Sources: GOC:TermGenie